{
  "term_id": "GO:0043235",
  "term_label": "receptor complex",
  "gene": "UniProtKB:Q99650",
  "gene_name": "Oncostatin-M-specific receptor subunit beta",
  "gene_symbol": "OSMR"
}